{
  "term_label": "Unknown biological process",
  "gene_name": "Zinc finger protein 831",
  "gene_symbol": "ZNF831",
  "term_id": "UNKNOWN:0002",
  "gene": "UniProtKB:Q5JPB2"
}